{
  "gene": "UniProtKB:A0A8V8TPE2",
  "gene_symbol": "FAM90A3P",
  "gene_name": "Family with sequence similarity 90 member A3, pseudogene",
  "term_label": "Unknown cellular component",
  "term_id": "UNKNOWN:0003"
}